{
  "gene": "UniProtKB:Q9NVM4",
  "gene_name": "Protein arginine N-methyltransferase 7",
  "gene_symbol": "PRMT7",
  "term_label": "chromatin remodeling",
  "term_id": "GO:0006338"
}